{
  "term_label": "RNA polymerase II cis-regulatory region sequence-specific DNA binding",
  "gene": "UniProtKB:P24278",
  "gene_name": "Zinc finger and BTB domain-containing protein 25",
  "gene_symbol": "ZBTB25",
  "term_id": "GO:0000978"
}